{
  "gene_name": "PH domain leucine-rich repeat-containing protein phosphatase 1",
  "gene": "UniProtKB:O60346",
  "term_label": "protein serine/threonine phosphatase activity",
  "gene_symbol": "PHLPP1",
  "term_id": "GO:0004722"
}